{
  "term_label": "Unknown molecular function",
  "gene_name": "Zyxin",
  "gene": "UniProtKB:Q15942",
  "term_id": "UNKNOWN:0001",
  "gene_symbol": "ZYX"
}